p-aminobenzoyl-glutamate transport [GO:0015814] (biological process) Definition: The directed movement of p-aminobenzoyl-glutamate, the anion of p-aminobenzoyl-glutamic acid, into, out of or within a cell, or between cells, by means of some agent such as a transporter or pore. Subtypes: p-aminobenzoyl-glutamate transmembrane transport [GO:1902604] Relationships: is a type of dicarboxylic acid transport [GO:0006835]; is_a GO:0042938; is a type of modified amino acid transport [GO:0072337] Sources: GOC:ai